{
  "term_label": "regulation of phosphatidylinositol 3-kinase/protein kinase B signal transduction",
  "gene": "UniProtKB:Q96T49",
  "gene_name": "Protein phosphatase 1 regulatory inhibitor subunit 16B",
  "gene_symbol": "PPP1R16B",
  "term_id": "GO:0051896"
}